L-mimosine synthase activity [GO:0050461] (molecular function) Definition: Catalysis of the reaction: 3,4-dihydroxypyridine + O-acetyl-L-serine = 3-(3,4-dihydroxypyridinium-1-yl)-L-alanine + acetate. Also known as: 3-O-acetyl-L-serine:3,4-dihydroxypyridine 1-(2-amino-2-carboxyethyl)transferase activity, O(3)-acetyl-L-serine acetate-lyase (adding 3,4-dihydroxypyridin-1-yl) activity, O3-acetyl-L-serine acetate-lyase (adding 3,4-dihydroxypyridin-1-yl), O3-acetyl-L-serine:3,4-dihydroxypyridine 1-(2-amino-2-carboxyethyl)transferase activity Sources: RHEA:12693 Relationships: is a type of transferase activity, transferring alkyl or aryl (other than methyl) groups [GO:0016765]